secondary alcohol metabolic process [GO:1902652] (biological process) References: PMID:11288200 Sources: GOC:TermGenie, GOC:mengo_curators, GO_REF:0000068 Subtypes: isocitrate metabolic process [GO:0006102], cholesterol metabolic process [GO:0008203], GO:0008204, GO:0008205, butanediol metabolic process [GO:0034077], zymosterol metabolic process [GO:0036196], GO:0045149, 6-sulfoquinovose(1-) catabolic process to glycerone phosphate and 3-sulfolactaldehyde [GO:0061720], vitamin D3 metabolic process [GO:0070640], asperfuranone catabolic process [GO:1900553], GO:1900580, secondary alcohol biosynthetic process [GO:1902653] Also known as: secondary alcohol metabolism Definition: The chemical reactions and pathways involving secondary alcohol. Relationships: is a type of alcohol metabolic process [GO:0006066]